{
  "gene_symbol": "TNFSF13",
  "term_label": "cytokine activity",
  "term_id": "GO:0005125",
  "gene_name": "Tumor necrosis factor ligand superfamily member 13",
  "gene": "UniProtKB:O75888"
}